{
  "term_id": "GO:0010468",
  "gene_symbol": "TRIM43",
  "term_label": "regulation of gene expression",
  "gene": "UniProtKB:Q96BQ3",
  "gene_name": "Tripartite motif-containing protein 43"
}